{
  "term_label": "Unknown molecular function",
  "term_id": "UNKNOWN:0001",
  "gene_symbol": "NPIPB15",
  "gene_name": "Nuclear pore complex-interacting protein family member B15",
  "gene": "UniProtKB:A6NHN6"
}